type IIa hypersensitivity [GO:0001794] (biological process) Definition: An inflammatory response resulting in cell death mediated by activation of the classical complement pathway or induction of effector cell phagocytosis or cytolysis mechanisms via complement or Fc receptors following the binding of antibodies to cell surface antigens on a target cell. Note: Note that some type IIb hypersensitivity responses (GO:0001795) are referred to simply as type II hypersensitivity in the earlier literature, but are mechanistically distinct from type IIa hypersensitivity. Sources: GOC:add, ISBN:0781735149 Subtypes: antibody-dependent cellular cytotoxicity [GO:0001788] Relationships: is a type of GO:0002445 Regulation: regulated by GO:0001796; negatively regulated by GO:0001797; positively regulated by positive regulation of type IIa hypersensitivity [GO:0001798]